{
  "gene_symbol": "CKMT1A",
  "term_label": "phosphocreatine biosynthetic process",
  "gene": "UniProtKB:P12532",
  "gene_name": "Creatine kinase U-type, mitochondrial",
  "term_id": "GO:0046314"
}